{
  "term_label": "cellular response to nitrogen starvation",
  "gene": "UniProtKB:Q14457",
  "gene_name": "Beclin-1",
  "gene_symbol": "BECN1",
  "term_id": "GO:0006995"
}